{
  "gene_symbol": "HSPA5",
  "gene_name": "Endoplasmic reticulum chaperone BiP",
  "term_label": "nucleus",
  "term_id": "GO:0005634",
  "gene": "UniProtKB:P11021"
}